capsule organization [GO:0045230] (biological process) Sources: GOC:ai Definition: A process that is carried out at the cellular level which results in the assembly, arrangement of constituent parts, or disassembly of the capsule, a protective structure surrounding some species of bacteria and fungi. Relationships: is a type of external encapsulating structure organization [GO:0045229] Subtypes: capsule polysaccharide biosynthetic process [GO:0045227], capsule poly-gamma-glutamate biosynthetic process [GO:0070502] Also known as: capsule organisation, capsule organization and biogenesis Regulation: regulated by GO:1901913; negatively regulated by negative regulation of capsule organization [GO:1901914]; positively regulated by positive regulation of capsule organization [GO:1901915]